{
  "term_id": "GO:0016485",
  "term_label": "protein processing",
  "gene_symbol": "ATG4A",
  "gene": "UniProtKB:Q8WYN0",
  "gene_name": "Cysteine protease ATG4A"
}